{
  "gene_symbol": "TMEM207",
  "gene_name": "Transmembrane protein 207",
  "term_id": "UNKNOWN:0002",
  "gene": "UniProtKB:Q6UWW9",
  "term_label": "Unknown biological process"
}